negative regulation of membrane protein ectodomain proteolysis [GO:0051045] (BP) Definition: Any process that stops, prevents, or reduces the frequency, rate or extent of membrane protein ectodomain proteolysis. Relationships: is a type of GO:0042177; is a type of negative regulation of proteolysis [GO:0045861]; is_a regulation of membrane protein ectodomain proteolysis [GO:0051043]; negatively regulates membrane protein ectodomain proteolysis [GO:0006509] Also known as: down regulation of membrane protein ectodomain proteolysis, down-regulation of membrane protein ectodomain proteolysis, downregulation of membrane protein ectodomain proteolysis, inhibition of membrane protein ectodomain proteolysis Sources: GOC:ai